{
  "gene": "UniProtKB:Q8NGZ2",
  "term_id": "GO:0005549",
  "gene_symbol": "OR14K1",
  "gene_name": "Olfactory receptor 14K1",
  "term_label": "odorant binding"
}